{
  "gene_symbol": "STK35",
  "term_label": "protein kinase activity",
  "term_id": "GO:0004672",
  "gene_name": "Serine_threonine-protein kinase 35",
  "gene": "UniProtKB:Q8TDR2"
}